{
  "term_id": "GO:0085029",
  "gene_symbol": "HAS2",
  "gene": "UniProtKB:Q92819",
  "term_label": "extracellular matrix assembly",
  "gene_name": "Hyaluronan synthase 2"
}